{
  "gene": "UniProtKB:A0A2Z4LIS9",
  "gene_name": "Forkhead box protein O3B",
  "term_id": "GO:0000978",
  "term_label": "RNA polymerase II cis-regulatory region sequence-specific DNA binding",
  "gene_symbol": "FOXO3B"
}